purinergic nucleotide receptor activity [GO:0001614] (molecular function) Also known as: purinoceptor, purinoreceptor, P2 receptor, purinergic receptor activity Sources: GOC:mah, GOC:signaling Definition: Combining with a purine nucleotide and transmitting the signal from one side of the membrane to the other to initiate a change in cell activity. Relationships: is a type of nucleotide receptor activity [GO:0016502]; is part of purinergic nucleotide receptor signaling pathway [GO:0035590]; has part purine nucleotide binding [GO:0017076] Subtypes: GO:0045028